regulation of blood-brain barrier permeability [GO:1905603] (biological process) References: PMID:22524708, PMID:30280653 Sources: GOC:TermGenie, GOC:als, GOC:aruk, GOC:bc, GO_REF:0000058 Relationships: is a type of regulation of vascular permeability [GO:0043114]; is part of maintenance of blood-brain barrier [GO:0035633] Also known as: regulation of BBB permeability, regulation of blood/brain barrier permeability Definition: Any process that modulates blood-brain barrier permeability, the quality of the blood-brain barrier that allows for a controlled passage of substances (e.g. macromolecules, small molecules, ions) into and out of the brain. Subtypes: negative regulation of blood-brain barrier permeability [GO:1905604], positive regulation of blood-brain barrier permeability [GO:1905605]